{
  "gene_symbol": "FRMPD2B",
  "gene": "UniProtKB:Q6IN97",
  "term_label": "Unknown molecular function",
  "term_id": "UNKNOWN:0001",
  "gene_name": "Putative protein FRMPD2-like"
}